{
  "gene": "UniProtKB:P40763",
  "gene_symbol": "STAT3",
  "term_id": "GO:0000981",
  "gene_name": "Signal transducer and activator of transcription 3",
  "term_label": "DNA-binding transcription factor activity, RNA polymerase II-specific"
}